{
  "gene": "UniProtKB:P49190",
  "term_label": "peptide hormone binding",
  "gene_symbol": "PTH2R",
  "term_id": "GO:0017046",
  "gene_name": "Parathyroid hormone 2 receptor"
}